{
  "gene_symbol": "GPC6",
  "term_label": "extracellular matrix",
  "gene": "UniProtKB:Q9Y625",
  "gene_name": "Glypican-6",
  "term_id": "GO:0031012"
}